{
  "gene_symbol": "HOXA2",
  "gene": "UniProtKB:O43364",
  "term_id": "GO:0006357",
  "term_label": "regulation of transcription by RNA polymerase II",
  "gene_name": "Homeobox protein Hox-A2"
}